regulation of iron-sulfur-molybdenum cofactor assembly [GO:1900506] (biological process) Definition: Any process that modulates the frequency, rate or extent of iron-sulfur-molybdenum cofactor assembly. Sources: GOC:TermGenie, GOC:mengo_curators Also known as: regulation of FeMoco assembly, regulation of FeMoco biosynthetic process, regulation of iron molybdenum cofactor assembly, regulation of iron molybdenum cofactor biosynthesis, regulation of iron molybdenum cofactor biosynthetic process Relationships: is a type of GO:1903329; regulates GO:0044593 Subtypes: negative regulation of iron-sulfur-molybdenum cofactor assembly [GO:1900507], positive regulation of iron-sulfur-molybdenum cofactor assembly [GO:1900508]